{
  "gene_symbol": "YDJC",
  "gene_name": "Carbohydrate deacetylase",
  "term_id": "GO:0019213",
  "gene": "UniProtKB:A8MPS7",
  "term_label": "deacetylase activity"
}